{
  "gene_symbol": "TNP1",
  "gene_name": "Spermatid nuclear transition protein 1",
  "gene": "UniProtKB:P09430",
  "term_id": "GO:0006338",
  "term_label": "chromatin remodeling"
}